{
  "gene_name": "Adipolin",
  "term_label": "positive regulation of D-glucose import",
  "gene_symbol": "C1QTNF12",
  "gene": "UniProtKB:Q5T7M4",
  "term_id": "GO:0046326"
}